{
  "term_id": "GO:0015379",
  "gene": "UniProtKB:Q9BXP2",
  "term_label": "potassium:chloride symporter activity",
  "gene_name": "Solute carrier family 12 member 9",
  "gene_symbol": "SLC12A9"
}